{
  "term_label": "signaling adaptor activity",
  "gene": "UniProtKB:Q8TEW6",
  "term_id": "GO:0035591",
  "gene_name": "Docking protein 4",
  "gene_symbol": "DOK4"
}